{
  "term_id": "GO:0008206",
  "gene_symbol": "AMACR",
  "gene": "UniProtKB:Q9UHK6",
  "term_label": "bile acid metabolic process",
  "gene_name": "Alpha-methylacyl-CoA racemase"
}